{
  "term_id": "GO:0005634",
  "term_label": "nucleus",
  "gene_name": "Melanoma-associated antigen F1",
  "gene_symbol": "MAGEF1",
  "gene": "UniProtKB:Q9HAY2"
}